{
  "gene_symbol": "PDLIM2",
  "term_label": "stress fiber",
  "gene": "UniProtKB:Q96JY6",
  "term_id": "GO:0001725",
  "gene_name": "PDZ and LIM domain protein 2"
}